isoflavone 4'-O-methyltransferase activity [GO:0030746] (MF) Also known as: 4'-hydroxyisoflavone methyltransferase activity, S-adenosyl-L-methionine:isoflavone 4'-O-methyltransferase activity, isoflavone O-methyltransferase activity, isoflavone methyltransferase activity Relationships: is a type of S-adenosylmethionine-dependent methyltransferase activity [GO:0008757] Sources: EC:2.1.1.46 Definition: Catalysis of the reaction: S-adenosyl-L-methionine + isoflavone = S-adenosyl-L-homocysteine + 4'-O-methylisoflavone.